{
  "gene": "UniProtKB:Q96H96",
  "term_id": "GO:0006744",
  "gene_symbol": "COQ2",
  "gene_name": "4-hydroxybenzoate polyprenyltransferase, mitochondrial",
  "term_label": "ubiquinone biosynthetic process"
}